{
  "term_label": "Unknown cellular component",
  "gene_symbol": "GPR162",
  "gene": "UniProtKB:Q16538",
  "gene_name": "Probable G-protein coupled receptor 162",
  "term_id": "UNKNOWN:0003"
}